{
  "term_id": "GO:0140658",
  "gene_name": "Chromodomain-helicase-DNA-binding protein 2",
  "term_label": "ATP-dependent chromatin remodeler activity",
  "gene": "UniProtKB:O14647",
  "gene_symbol": "CHD2"
}